{
  "gene_symbol": "RSPH9",
  "gene_name": "Radial spoke head protein 9 homolog",
  "term_label": "motile cilium assembly",
  "term_id": "GO:0044458",
  "gene": "UniProtKB:Q9H1X1"
}